{
  "gene_name": "5-hydroxytryptamine receptor 3A",
  "term_label": "monoatomic ion transmembrane transport",
  "term_id": "GO:0034220",
  "gene": "UniProtKB:P46098",
  "gene_symbol": "HTR3A"
}